{
  "gene_symbol": "CPS1",
  "gene": "UniProtKB:P31327",
  "gene_name": "Carbamoyl-phosphate synthase [ammonia], mitochondrial",
  "term_id": "GO:0006541",
  "term_label": "glutamine metabolic process"
}